{
  "gene_symbol": "KATNAL1",
  "gene": "UniProtKB:Q9BW62",
  "gene_name": "Katanin p60 ATPase-containing subunit A-like 1",
  "term_label": "microtubule severing ATPase activity",
  "term_id": "GO:0008568"
}